{
  "term_id": "GO:0007204",
  "term_label": "positive regulation of cytosolic calcium ion concentration",
  "gene": "UniProtKB:O00421",
  "gene_name": "C-C chemokine receptor-like 2",
  "gene_symbol": "CCRL2"
}